{
  "term_label": "Unknown cellular component",
  "gene_symbol": "CCDC71L",
  "gene": "UniProtKB:Q8N9Z2",
  "term_id": "UNKNOWN:0003",
  "gene_name": "Coiled-coil domain-containing protein 71L"
}